{
  "gene_name": "Actin-histidine N-methyltransferase",
  "term_label": "transcription coactivator activity",
  "gene": "UniProtKB:Q86TU7",
  "gene_symbol": "SETD3",
  "term_id": "GO:0003713"
}